{
  "gene_name": "Caspase-14",
  "gene": "UniProtKB:P31944",
  "term_id": "GO:0043525",
  "term_label": "positive regulation of neuron apoptotic process",
  "gene_symbol": "CASP14"
}